{
  "gene": "UniProtKB:Q9GZR2",
  "gene_name": "RNA exonuclease 4",
  "term_id": "GO:0005634",
  "gene_symbol": "REXO4",
  "term_label": "nucleus"
}